{
  "gene_name": "Small cysteine and glycine repeat-containing protein 7",
  "term_label": "Unknown cellular component",
  "term_id": "UNKNOWN:0003",
  "gene": "UniProtKB:A0A286YF01",
  "gene_symbol": "SCYGR7"
}